{
  "gene_name": "Endosome_lysosome-associated apoptosis and autophagy regulator family member 2",
  "term_label": "positive regulation of BMP signaling pathway",
  "gene": "UniProtKB:A8MWY0",
  "gene_symbol": "ELAPOR2",
  "term_id": "GO:0030513"
}